{
  "term_label": "sister chromatid cohesion",
  "gene": "UniProtKB:Q8NDV3",
  "gene_name": "Structural maintenance of chromosomes protein 1B",
  "term_id": "GO:0007062",
  "gene_symbol": "SMC1B"
}